zeatin O-beta-D-xylosyltransferase activity [GO:0050404] (molecular function) Sources: EC:2.4.2.40, RHEA:14721 Definition: Catalysis of the reaction: UDP-alpha-D-xylose + zeatin = O-beta-D-xylosylzeatin + H+ + UDP. Relationships: is a type of UDP-xylosyltransferase activity [GO:0035252] Also known as: zeatin O-b-D-xylosyltransferase activity, UDP-D-xylose:zeatin O-beta-D-xylosyltransferase activity, uridine diphosphoxylose-zeatin xylosyltransferase activity, zeatin O-xylosyltransferase activity